{
  "gene": "UniProtKB:Q8NCT3",
  "term_id": "UNKNOWN:0002",
  "term_label": "Unknown biological process",
  "gene_name": "Putative tyrosine carboxypeptidase MATCAP2",
  "gene_symbol": "MATCAP2"
}